{
  "term_id": "GO:0048678",
  "gene": "UniProtKB:Q8NDC4",
  "term_label": "response to axon injury",
  "gene_name": "MORN repeat-containing protein 4",
  "gene_symbol": "MORN4"
}